{
  "gene_symbol": "SEZ6",
  "term_label": "Unknown molecular function",
  "gene_name": "Seizure protein 6 homolog",
  "gene": "UniProtKB:Q53EL9",
  "term_id": "UNKNOWN:0001"
}